protein-glucosylgalactosylhydroxylysine glucosidase activity [GO:0047402] (molecular function) Sources: EC:3.2.1.107, MetaCyc:3.2.1.107-RXN Relationships: is a type of glucosidase activity [GO:0015926]; is a type of catalytic activity, acting on a protein [GO:0140096] Definition: Catalysis of the reaction: H2O + protein alpha-D-glucosyl-1,2-beta-D-galactosyl-L-hydroxylysine = protein beta-D-galactosyl-L-hydroxylysine + beta-D-glucose. The enzyme specifically hydrolyzes glucose from alpha-D-glucosyl- (1->2)-beta-D-galactosyl disaccharide units that are linked to hydroxylysine residues of collagen and collagen-like proteins. Also known as: 2-O-alpha-D-glucopyranosyl-5-O-alpha-D-galactopyranosylhydroxy-L-lysine glucohydrolase activity, protein-alpha-D-glucosyl-1,2-beta-D-galactosyl-L-hydroxylysine glucohydrolase activity